protein-cysteine S-myristoyltransferase activity [GO:0019705] (MF) Relationships: is a type of myristoyltransferase activity [GO:0019107]; is a type of protein-cysteine S-acyltransferase activity [GO:0019707] References: PMID:22247542 Sources: GOC:ai, RHEA:59736 Definition: Catalysis of the transfer of a myristoyl (systematic name, tetradecanoyl) group to a sulfur atom on a cysteine residue of a protein molecule in the reaction: tetradecanoyl-CoA + L-cysteinyl-[protein] = CoA + S-tetradecanoyl-L-cysteinyl-[protein].